{
  "term_id": "GO:0005886",
  "term_label": "plasma membrane",
  "gene_name": "Glycerophosphoinositol inositolphosphodiesterase GDPD2",
  "gene_symbol": "GDPD2",
  "gene": "UniProtKB:Q9HCC8"
}